{
  "gene": "UniProtKB:Q14761",
  "gene_name": "Protein tyrosine phosphatase receptor type C-associated protein",
  "term_id": "UNKNOWN:0001",
  "term_label": "Unknown molecular function",
  "gene_symbol": "PTPRCAP"
}